regulation of systemic arterial blood pressure [GO:0003073] (biological process) Subtypes: GO:0002530, GO:0003044, regulation of systemic arterial blood pressure by physical factors [GO:0003045], circadian regulation of systemic arterial blood pressure [GO:0003052], GO:1900133 Relationships: is a type of regulation of blood pressure [GO:0008217] Sources: GOC:mtg_cardio Definition: The process that modulates the force with which blood travels through the systemic arterial circulatory system. The process is controlled by a balance of processes that increase pressure and decrease pressure.